{
  "term_label": "cytoplasm",
  "gene_name": "Caveolae-associated protein 1",
  "gene_symbol": "CAVIN1",
  "term_id": "GO:0005737",
  "gene": "UniProtKB:Q6NZI2"
}